{
  "gene_name": "Fragile X messenger ribonucleoprotein 1",
  "gene_symbol": "FMR1",
  "term_label": "mRNA 3'-UTR binding",
  "term_id": "GO:0003730",
  "gene": "UniProtKB:Q06787"
}